{
  "gene_symbol": "ZPBP2",
  "gene": "UniProtKB:Q6X784",
  "term_id": "GO:0002199",
  "gene_name": "Zona pellucida-binding protein 2",
  "term_label": "zona pellucida receptor complex"
}